{
  "term_label": "nucleus",
  "term_id": "GO:0005634",
  "gene": "UniProtKB:P13631",
  "gene_name": "Retinoic acid receptor gamma",
  "gene_symbol": "RARG"
}